{
  "gene": "UniProtKB:P0DW14",
  "gene_symbol": "TAF11L10",
  "term_label": "transcription factor TFIID complex",
  "gene_name": "TATA-box-binding protein-associated factor 11-like protein 10",
  "term_id": "GO:0005669"
}